symbiont-mediated activation of host apoptosis [GO:0052151] (biological process) Note: Note that term is to be used to annotate gene products in the symbiont that play an active role in the activation of host apoptosis, usually by directly activating molecules involved either in apoptotic signaling or in apoptosis (such as caspases). Proteins and other molecules detected by the host that trigger host apoptosis should not be annotated to this term. Also known as: activation by organism of host apoptosis, activation by organism of host apoptotic programmed cell death, induction by organism of host apoptotic programmed cell death, induction by symbiont of host apoptosis, positive regulation by organism of host apoptotic programmed cell death, positive regulation by symbiont of host apoptotic process, up regulation by organism of host apoptotic programmed cell death, up regulation by symbiont of host apoptosis, up-regulation by organism of host apoptotic programmed cell death, up-regulation by symbiont of host apoptosis, upregulation by organism of host apoptotic programmed cell death, upregulation by symbiont of host apoptosis, activation by symbiont of host apoptosis, positive regulation by symbiont of host apoptosis, positive regulation by virus of host apoptosis, stimulation by symbiont of host apoptosis References: PMID:11805081, PMID:18037263, PMID:19801898, PMID:29571981 Relationships: is_a symbiont-mediated killing of host cell [GO:0001907]; is a type of symbiont-mediated activation of host programmed cell death [GO:0052042]; is a type of GO:0052150 Definition: A process in which a symbiont initiates, promotes, or enhances the normal execution of host apoptosis, leading to an increase in the frequency, rate or extent of apoptosis in the host cell. The host is defined as the larger of the organisms involved in a symbiotic interaction.